{
  "term_label": "regulation of DNA-templated transcription",
  "gene": "UniProtKB:Q9UGL1",
  "term_id": "GO:0006355",
  "gene_symbol": "KDM5B",
  "gene_name": "Lysine-specific demethylase 5B"
}